{
  "gene": "UniProtKB:Q86XI6",
  "term_label": "glycogen binding",
  "gene_name": "Protein phosphatase 1 regulatory subunit 3B",
  "term_id": "GO:2001069",
  "gene_symbol": "PPP1R3B"
}